{
  "term_label": "RNA endonuclease activity",
  "gene": "UniProtKB:Q53H82",
  "gene_name": "Endoribonuclease LACTB2",
  "term_id": "GO:0004521",
  "gene_symbol": "LACTB2"
}